{
  "gene_symbol": "PDZD4",
  "term_label": "Unknown biological process",
  "gene_name": "PDZ domain-containing protein 4",
  "term_id": "UNKNOWN:0002",
  "gene": "UniProtKB:Q76G19"
}